phosphatidylethanolamine acyl-chain remodeling [GO:0036152] (biological process) Relationships: is a type of phosphatidylcholine metabolic process [GO:0046470] References: PMID:18287005, PMID:18458083 Sources: GOC:mw Also known as: phosphatidylethanolamine acyl-chain remodelling Definition: Remodeling the acyl chains of phosphatidylethanolamine, through sequential deacylation and re-acylation reactions, to generate phosphatidylethanolamine containing different types of fatty acid acyl chains.